{
  "gene_name": "XK-related protein 8",
  "term_label": "plasma membrane",
  "gene_symbol": "XKR8",
  "gene": "UniProtKB:Q9H6D3",
  "term_id": "GO:0005886"
}